chemotaxis to arachidonate [GO:0034670] (biological process) Also known as: chemotaxis to arachidonic acid Definition: The directed movement of a motile cell or organism in response to the presence of arachidonic acid. Relationships: is a type of chemotaxis [GO:0006935] References: PMID:18202452 Sources: GOC:go_curators Regulation: regulated by regulation of chemotaxis to arachidonate [GO:1904552]; negatively regulated by negative regulation of chemotaxis to arachidonate [GO:1904553]; positively regulated by positive regulation of chemotaxis to arachidonate [GO:1904554]